{
  "gene_name": "Uncharacterized protein C2orf66",
  "term_id": "UNKNOWN:0001",
  "gene_symbol": "C2orf66",
  "term_label": "Unknown molecular function",
  "gene": "UniProtKB:Q6UXQ4"
}